acyl-CoA dehydrogenase (NADP+) activity [GO:0047616] (MF) Definition: Catalysis of the reaction: acyl-CoA + NADP+ = 2,3-dehydroacyl-CoA + NADPH + H+. Relationships: is a type of oxidoreductase activity, acting on the CH-CH group of donors, NAD or NADP as acceptor [GO:0016628] Sources: EC:1.3.1.8 Also known as: 2-enoyl-CoA reductase activity, acyl-CoA:NADP+ 2-oxidoreductase activity, crotonyl coenzyme A reductase activity, dehydrogenase, acyl coenzyme A (nicotinamide adenine dinucleotide phosphate), enoyl coenzyme A reductase activity